{
  "gene_name": "Prostate and testis expressed protein 2",
  "gene_symbol": "PATE2",
  "gene": "UniProtKB:Q6UY27",
  "term_id": "UNKNOWN:0001",
  "term_label": "Unknown molecular function"
}